{
  "gene_symbol": "PPP2R1A",
  "term_label": "cytoplasm",
  "gene": "UniProtKB:P30153",
  "term_id": "GO:0005737",
  "gene_name": "Serine_threonine-protein phosphatase 2A 65 kDa regulatory subunit A alpha isoform"
}